embryonic axis specification [GO:0000578] (biological process) Definition: The establishment, maintenance and elaboration of a pattern along a line or a point in an embryo. Sources: GOC:dph, GOC:go_curators, GOC:sdb_2009, GOC:tb Subtypes: zygotic specification of dorsal/ventral axis [GO:0007352], GO:0008595, longitudinal axis specification [GO:0009942], GO:0021997, GO:0032525, oral/aboral axis specification [GO:0060834] Also known as: embryonic axis determination Relationships: is a type of axis specification [GO:0009798]; is a type of embryonic pattern specification [GO:0009880]